{
  "gene_name": "Putative uncharacterized protein PP6455",
  "term_label": "Unknown cellular component",
  "term_id": "UNKNOWN:0003",
  "gene_symbol": "PP6455",
  "gene": "UniProtKB:Q8WZ26"
}